{
  "gene_name": "Uridine-cytidine kinase-like 1",
  "term_id": "GO:0004849",
  "gene_symbol": "UCKL1",
  "gene": "UniProtKB:Q9NWZ5",
  "term_label": "uridine kinase activity"
}